{
  "term_label": "G protein-coupled receptor signaling pathway",
  "gene_symbol": "GPR142",
  "gene_name": "Probable G-protein coupled receptor 142",
  "term_id": "GO:0007186",
  "gene": "UniProtKB:Q7Z601"
}